{
  "gene_symbol": "AGO1",
  "gene": "UniProtKB:Q9UL18",
  "gene_name": "Protein argonaute-1",
  "term_label": "cytoplasmic ribonucleoprotein granule",
  "term_id": "GO:0036464"
}